{
  "gene": "UniProtKB:Q9BZM6",
  "term_id": "GO:0002476",
  "gene_symbol": "ULBP1",
  "term_label": "antigen processing and presentation of endogenous peptide antigen via MHC class Ib",
  "gene_name": "UL16-binding protein 1"
}